{
  "gene_name": "AN1-type zinc finger protein 6",
  "term_label": "Unknown cellular component",
  "term_id": "UNKNOWN:0003",
  "gene": "UniProtKB:Q6FIF0",
  "gene_symbol": "ZFAND6"
}